response to methylmercury [GO:0051597] (biological process) Definition: Any process that results in a change in state or activity of a cell or an organism (in terms of movement, secretion, enzyme production, gene expression, etc.) as a result of a methylmercury stimulus. Subtypes: cellular response to methylmercury [GO:0071406] Sources: GOC:ai Relationships: is_a response to chemical [GO:0042221] Also known as: response to CH3-Hg+, response to MeHg+